{
  "term_label": "nucleus",
  "term_id": "GO:0005634",
  "gene_name": "Endothelial differentiation-related factor 1",
  "gene": "UniProtKB:O60869",
  "gene_symbol": "EDF1"
}